{
  "gene_symbol": "AQP12B",
  "gene": "UniProtKB:A6NM10",
  "gene_name": "Aquaporin-12B",
  "term_id": "GO:0015267",
  "term_label": "channel activity"
}